{
  "term_label": "neuron projection",
  "term_id": "GO:0043005",
  "gene": "UniProtKB:Q96EV8",
  "gene_symbol": "DTNBP1",
  "gene_name": "Dysbindin"
}